{
  "term_id": "GO:0042056",
  "gene_name": "Vascular endothelial growth factor D",
  "term_label": "chemoattractant activity",
  "gene_symbol": "VEGFD",
  "gene": "UniProtKB:O43915"
}